{
  "gene_symbol": "ATG9B",
  "term_label": "phospholipid scramblase activity",
  "gene_name": "Autophagy-related protein 9B",
  "gene": "UniProtKB:Q674R7",
  "term_id": "GO:0017128"
}